quercetin-3-sulfate 4'-sulfotransferase activity [GO:0047366] (molecular function) Sources: EC:2.8.2.27, RHEA:17205 Definition: Catalysis of the reaction: 3'-phospho-5'-adenylyl sulfate + quercetin 3-sulfate = adenosine 3',5'-diphosphate + H+ + quercetin 3,4'-disulfate. Relationships: is a type of sulfotransferase activity [GO:0008146] Also known as: quercetin-3-sulphate 4'-sulphotransferase activity, 3'-phosphoadenylyl-sulfate:quercetin-3-sulfate 4'-sulfotransferase activity, PAPS:flavonol 3-sulfate 4'-sulfotransferase activity, flavonol 4'-sulfotransferase activity